{
  "gene_name": "Inhibitor of nuclear factor kappa-B kinase subunit beta",
  "term_id": "GO:0008385",
  "term_label": "IkappaB kinase complex",
  "gene_symbol": "IKBKB",
  "gene": "UniProtKB:O14920"
}